{
  "gene_symbol": "PRXL2C",
  "term_label": "Unknown biological process",
  "gene_name": "Peroxiredoxin-like 2C",
  "term_id": "UNKNOWN:0002",
  "gene": "UniProtKB:Q7RTV5"
}